urea channel activity [GO:0015265] (molecular function) Definition: Enables the energy-independent facilitated diffusion of urea through a transmembrane aqueous pore or channel. Relationships: is a type of urea transmembrane transporter activity [GO:0015204]; is a type of GO:0015267 Sources: GOC:mtg_transport